{
  "gene": "UniProtKB:Q9H1K1",
  "gene_name": "Iron-sulfur cluster assembly enzyme ISCU",
  "term_id": "GO:0005737",
  "gene_symbol": "ISCU",
  "term_label": "cytoplasm"
}